{
  "term_label": "glutathione metabolic process",
  "term_id": "GO:0006749",
  "gene_name": "Glutathione S-transferase omega-1",
  "gene": "UniProtKB:P78417",
  "gene_symbol": "GSTO1"
}